vesicle-mediated transport between endosomal compartments [GO:0098927] (biological process) Subtypes: GO:0045022, early endosome to recycling endosome transport [GO:0061502] Definition: A cellular transport process in which transported substances are moved in membrane-bounded vesicles between endosomal compartments, e.g, between early endosome and sorting endosome. References: PMID:10930469 Sources: GOC:dos Relationships: is a type of endosomal transport [GO:0016197]